{
  "term_id": "GO:0005737",
  "gene_symbol": "CDKN3",
  "gene": "UniProtKB:Q16667",
  "term_label": "cytoplasm",
  "gene_name": "Cyclin-dependent kinase inhibitor 3"
}